{
  "term_id": "GO:0019901",
  "term_label": "protein kinase binding",
  "gene_symbol": "RHOH",
  "gene_name": "Rho-related GTP-binding protein RhoH",
  "gene": "UniProtKB:Q15669"
}